{
  "term_label": "putrescine biosynthetic process from arginine, via ornithine",
  "gene_name": "Antizyme inhibitor 1",
  "gene_symbol": "AZIN1",
  "gene": "UniProtKB:O14977",
  "term_id": "GO:0033387"
}